{
  "term_id": "UNKNOWN:0002",
  "gene_symbol": "LORICRIN",
  "term_label": "Unknown biological process",
  "gene": "UniProtKB:P23490",
  "gene_name": "Loricrin"
}